{
  "gene_name": "DNA-directed RNA polymerase, mitochondrial",
  "gene_symbol": "POLRMT",
  "term_id": "GO:0034245",
  "term_label": "mitochondrial DNA-directed RNA polymerase complex",
  "gene": "UniProtKB:O00411"
}